N-acetylglucosaminylinositol deacetylase activity [GO:0035595] (molecular function) Sources: RHEA:26180 Relationships: is a type of hydrolase activity, acting on carbon-nitrogen (but not peptide) bonds, in linear amides [GO:0016811]; is a type of deacetylase activity [GO:0019213] Also known as: GlcNAc-Ins deacetylase activity, 1-(2-acetamido-2-deoxy-alpha-D-glucopyranosyl)-1D-myo-inositol acetylhydrolase activity, 1D-myo-inositol 2-acetamido-2-deoxy-alpha-D-glucopyranoside deacetylase activity, N-acetyl-1D-myo-inositol-2-amino-2-deoxy-alpha-D-glucopyranoside deacetylase activity Definition: Catalysis of the reaction: 1D-myo-inositol 2-acetamido-2-deoxy-alpha-D-glucopyranoside + H2O = 1D-myo-inositol 2-amino-2-deoxy-alpha-D-glucopyranoside + acetate. This reaction is the hydrolysis of an acetyl group from N-acetylglucosaminylinositol.